{
  "gene": "UniProtKB:P05556",
  "gene_name": "Integrin beta-1",
  "term_label": "cell surface",
  "gene_symbol": "ITGB1",
  "term_id": "GO:0009986"
}